transverse flagellum [GO:0097608] (cellular component) Also known as: transverse cilium Note: Note that we deem cilium and microtubule-based flagellum to be equivalent. In this case community usage refers to 'flagellum' rather than 'cilium', hence the primary term name, but the cilium parentage is deliberate. Sources: GOC:at, Wikipedia:Dinoflagellate#Morphology, http://tolweb.org/Dinoflagellates/2445, https://doi.org/10.1038/213421a0 Relationships: is a type of 9+2 motile cilium [GO:0097729] Definition: A motile cilium found in dinoflagellates. It coils around the cell and provides the forward thrust for motility. It is often contained in a furrow called the cingulum, and emerges from a flagellar pore located in the cingulum.